{
  "term_label": "RNA polymerase II cis-regulatory region sequence-specific DNA binding",
  "term_id": "GO:0000978",
  "gene": "UniProtKB:P14653",
  "gene_name": "Homeobox protein Hox-B1",
  "gene_symbol": "HOXB1"
}